{
  "term_label": "inositol tetrakisphosphate kinase activity",
  "gene": "UniProtKB:Q8NFU5",
  "term_id": "GO:0051765",
  "gene_name": "Inositol polyphosphate multikinase",
  "gene_symbol": "IPMK"
}